regulation of homologous chromosome segregation [GO:0060629] (BP) Definition: Any process that modulates the rate, frequency, or extent of homologous chromosome segregation, the cell cycle process in which replicated homologous chromosomes are organized and then physically separated and apportioned to two sets during the first division of the meiotic cell cycle. Each replicated chromosome, composed of two sister chromatids, aligns at the cell equator, paired with its homologous partner; this pairing off, referred to as synapsis, permits genetic recombination. One homolog (both sister chromatids) of each morphologic type goes into each of the resulting chromosome sets. Relationships: is a type of GO:0051983; is a type of GO:2000241; regulates GO:0045143 Subtypes: regulation of linear element assembly [GO:0090006] Sources: GOC:dph, GOC:tb